{
  "term_id": "GO:0048666",
  "gene": "UniProtKB:O14813",
  "term_label": "neuron development",
  "gene_name": "Paired mesoderm homeobox protein 2A",
  "gene_symbol": "PHOX2A"
}